dystrophin-associated glycoprotein complex [GO:0016010] (cellular component) Relationships: is a type of glycoprotein complex [GO:0090665]; is_a plasma membrane protein complex [GO:0098797] Also known as: DGC, dystrophin glycoprotein complex Definition: A multiprotein complex that forms a strong mechanical link between the cytoskeleton and extracellular matrix; typical of, but not confined to, muscle cells. The complex is composed of transmembrane, cytoplasmic, and extracellular proteins, including dystrophin, sarcoglycans, dystroglycan, dystrobrevins, syntrophins, sarcospan, caveolin-3, and NO synthase. References: PMID:15117830, PMID:16710609